{
  "gene": "UniProtKB:P98095",
  "gene_symbol": "FBLN2",
  "term_id": "GO:0005576",
  "term_label": "extracellular region",
  "gene_name": "Fibulin-2"
}